DNA topoisomerase type II (double strand cut, ATP-hydrolyzing) activator activity [GO:0072587] (molecular function) Definition: Binds to and increases the activity of ATP-hydrolyzing DNA topoisomerase. DNA topoisomerase (ATP-hydrolyzing) regulator activity catalyzes a DNA topological transformation by transiently cleaving a pair of complementary DNA strands to form a gate through which a second double-stranded DNA segment is passed, after which the severed strands in the first DNA segment are rejoined; product release is coupled to ATP binding and hydrolysis; changes the linking number in multiples of 2. Sources: GOC:mah Relationships: is a type of ATPase activator activity [GO:0001671]; is_a enzyme activator activity [GO:0008047]; is a type of DNA topoisomerase type II (double strand cut, ATP-hydrolyzing) regulator activity [GO:0072586]; positively regulates DNA topoisomerase type II (double strand cut, ATP-hydrolyzing) activity [GO:0003918]